inositol-1,3,4-trisphosphate 4-phosphatase activity [GO:0017161] (molecular function) Sources: GOC:ai Relationships: is_a GO:0046030 Definition: Catalysis of the reaction: D-myo-inositol 1,3,4-trisphosphate + H2O = myo-inositol 1,3-bisphosphate + phosphate.